{
  "gene": "UniProtKB:Q99788",
  "term_label": "positive regulation of macrophage chemotaxis",
  "gene_symbol": "CMKLR1",
  "term_id": "GO:0010759",
  "gene_name": "Chemerin-like receptor 1"
}